{
  "gene_symbol": "ADAM28",
  "gene": "UniProtKB:Q9UKQ2",
  "term_id": "GO:0006508",
  "term_label": "proteolysis",
  "gene_name": "Disintegrin and metalloproteinase domain-containing protein 28"
}